{
  "gene": "UniProtKB:Q8TCE6",
  "gene_symbol": "DENND10",
  "term_id": "GO:0015031",
  "term_label": "protein transport",
  "gene_name": "DENN domain-containing protein 10"
}